{
  "gene": "UniProtKB:Q6ZSA8",
  "term_id": "UNKNOWN:0003",
  "gene_name": "Putative uncharacterized protein FLJ45684",
  "term_label": "Unknown cellular component",
  "gene_symbol": "Q6ZSA8"
}